site-specific recombinase activity [GO:0009009] (molecular function) Note: Note that this term is not a child of 'recombinase activity ; GO:0000150' because the latter represents activities that do not break or form phosphodiester bonds. Definition: Catalysis of the formation of new phosphodiester bonds between a pair of short, unique target DNA sequences. Also known as: RecA-family recombinase activity Relationships: is a type of integrase activity [GO:0008907] Subtypes: GO:0008979, GO:0009037, serine-based site-specific recombinase activity [GO:0160053] References: PMID:6286142 Sources: GOC:elh